{
  "term_label": "Unknown cellular component",
  "gene_name": "LBH domain-containing protein 2",
  "gene": "UniProtKB:A0A0U1RRK4",
  "term_id": "UNKNOWN:0003",
  "gene_symbol": "LBHD2"
}